{
  "gene": "UniProtKB:A0A1B0GVS7",
  "gene_name": "MyoD family inhibitor domain-containing protein 2",
  "gene_symbol": "MDFIC2",
  "term_label": "Unknown molecular function",
  "term_id": "UNKNOWN:0001"
}